{
  "gene_symbol": "OR4C6",
  "term_id": "UNKNOWN:0002",
  "term_label": "Unknown biological process",
  "gene_name": "Olfactory receptor 4C6",
  "gene": "UniProtKB:Q8NH72"
}